glutamine synthetase activity [GO:0004356] (molecular function) Relationships: is a type of ammonia ligase activity [GO:0016211] Also known as: glutamate-ammonia ligase activity, L-glutamine synthetase activity Definition: Catalysis of the reaction: ATP + L-glutamate + NH4+ = ADP + H+ + L-glutamine + phosphate. Sources: RHEA:16169